{
  "gene": "UniProtKB:Q9BYT9",
  "term_id": "GO:0005886",
  "gene_symbol": "ANO3",
  "gene_name": "Anoctamin-3",
  "term_label": "plasma membrane"
}